{
  "term_id": "UNKNOWN:0002",
  "gene_symbol": "CNPY4",
  "gene": "UniProtKB:Q8N129",
  "gene_name": "Protein canopy homolog 4",
  "term_label": "Unknown biological process"
}